{
  "term_label": "male germ cell nucleus",
  "gene_symbol": "SYCP1",
  "gene_name": "Synaptonemal complex protein 1",
  "term_id": "GO:0001673",
  "gene": "UniProtKB:Q15431"
}